{
  "term_id": "GO:0016992",
  "gene": "UniProtKB:O43766",
  "gene_name": "Lipoyl synthase, mitochondrial",
  "term_label": "lipoate synthase activity",
  "gene_symbol": "LIAS"
}